negative regulation of collecting lymphatic vessel constriction [GO:1903815] (biological process) References: PMID:23897233 Sources: GOC:TermGenie, GO_REF:0000058 Relationships: is a type of negative regulation of multicellular organismal process [GO:0051241]; is a type of regulation of collecting lymphatic vessel constriction [GO:1903814]; negatively regulates collecting lymphatic vessel constriction [GO:1990192] Also known as: down regulation of collecting lymphatic vessel constriction, down regulation of lymphatic vessel myogenic constriction, down-regulation of collecting lymphatic vessel constriction, down-regulation of lymphatic vessel myogenic constriction, downregulation of collecting lymphatic vessel constriction, downregulation of lymphatic vessel myogenic constriction, negative regulation of lymphatic vessel myogenic constriction, inhibition of collecting lymphatic vessel constriction, inhibition of lymphatic vessel myogenic constriction Definition: Any process that stops, prevents or reduces the frequency, rate or extent of collecting lymphatic vessel constriction.